{
  "gene": "UniProtKB:Q9BRU9",
  "gene_symbol": "UTP23",
  "gene_name": "rRNA-processing protein UTP23 homolog",
  "term_id": "GO:0005730",
  "term_label": "nucleolus"
}